sterol biosynthetic process [GO:0016126] (biological process) Sources: GOC:go_curators Regulation: regulated by regulation of sterol biosynthetic process [GO:0106118]; RO_0002212 by negative regulation of sterol biosynthetic process [GO:0106119]; positively regulated by GO:0106120 Subtypes: cholesterol biosynthetic process [GO:0006695], ergosterol biosynthetic process [GO:0006696], ecdysone biosynthetic process [GO:0006697], zymosterol biosynthetic process [GO:0036197] Definition: The chemical reactions and pathways resulting in the formation of sterols, steroids with one or more hydroxyl groups and a hydrocarbon side-chain in the molecule. Relationships: is a type of steroid biosynthetic process [GO:0006694]; is a type of sterol metabolic process [GO:0016125] Also known as: sterol anabolism, sterol biosynthesis, sterol formation, sterol synthesis